negative regulation of polyketide biosynthetic process [GO:1900733] (biological process) Definition: Any process that stops, prevents or reduces the frequency, rate or extent of polyketide biosynthetic process. Sources: GOC:TermGenie, GOC:di Also known as: down regulation of polyketide anabolism, down regulation of polyketide biosynthesis, down regulation of polyketide biosynthetic process, down regulation of polyketide formation, down regulation of polyketide synthesis, down-regulation of polyketide anabolism, down-regulation of polyketide biosynthesis, down-regulation of polyketide biosynthetic process, down-regulation of polyketide formation, down-regulation of polyketide synthesis, downregulation of polyketide anabolism, downregulation of polyketide biosynthesis, downregulation of polyketide biosynthetic process, downregulation of polyketide formation, downregulation of polyketide synthesis, inhibition of polyketide anabolism, inhibition of polyketide biosynthesis, inhibition of polyketide formation, inhibition of polyketide synthesis, negative regulation of polyketide anabolism, negative regulation of polyketide biosynthesis, negative regulation of polyketide formation, negative regulation of polyketide synthesis, inhibition of polyketide biosynthetic process Relationships: is_a GO:1900377; is a type of regulation of polyketide biosynthetic process [GO:1900732]; negatively regulates polyketide biosynthetic process [GO:0030639] Subtypes: negative regulation of asperfuranone biosynthetic process [GO:1900638], GO:1900671, GO:1900676, negative regulation of neosartoricin biosynthetic process [GO:1902054]